{
  "gene_symbol": "SELENOV",
  "term_id": "GO:0005829",
  "gene_name": "Selenoprotein V",
  "term_label": "cytosol",
  "gene": "UniProtKB:P59797"
}